{
  "gene_symbol": "MLANA",
  "gene_name": "Melanoma antigen recognized by T-cells 1",
  "term_id": "GO:0005802",
  "gene": "UniProtKB:Q16655",
  "term_label": "trans-Golgi network"
}